dihydroneopterin triphosphate 2'-epimerase activity [GO:0008719] (molecular function) Relationships: is a type of racemase and epimerase activity [GO:0016854] Definition: Catalysis of the reaction: 7,8-dihydroneopterin 3'-triphosphate = 7,8-dihydromonapterin 3'-triphosphate. Sources: RHEA:28346 Also known as: D-erythro-7,8-dihydroneopterin triphosphate 2'-epimerase activity